{
  "gene_name": "Protein Shroom3",
  "term_id": "GO:0043296",
  "gene": "UniProtKB:Q8TF72",
  "gene_symbol": "SHROOM3",
  "term_label": "apical junction complex"
}